nitrogen compound transport [GO:0071705] (biological process) Definition: The directed movement of nitrogen-containing compounds into, out of or within a cell, or between cells, by means of some agent such as a transporter or pore. Relationships: is a type of transport [GO:0006810] Subtypes: sulfur amino acid transport [GO:0000101], beta-alanine transport [GO:0001762], asparagine transport [GO:0006867], glutamine transport [GO:0006868], glutamate secretion [GO:0014047], protein transport [GO:0015031], GO:0015686, GO:0015697, cyanate transport [GO:0015704], GO:0015707, bilirubin transport [GO:0015723], GO:0015734, GO:0015747, aromatic amino acid transport [GO:0015801], GO:0015803, GO:0015807, aspartate transmembrane transport [GO:0015810], gamma-aminobutyric acid transport [GO:0015812], GO:0015816, ornithine transport [GO:0015822], phenylalanine transport [GO:0015823], threonine transport [GO:0015826], GO:0015830, GO:0015835, amine transport [GO:0015837], cadaverine transport [GO:0015839], monoamine transport [GO:0015844], polyamine transport [GO:0015846], nucleobase transport [GO:0015851], acetylcholine transport [GO:0015870], choline transport [GO:0015871], biopterin transport [GO:0015877], GO:0015886, thiamine transport [GO:0015888], GO:0015889, aminotriazole transport [GO:0015899], fluconazole transport [GO:0015903], GO:0015905, aminophospholipid transport [GO:0015917], GO:0015931, GO:0030185, vitamin B6 transport [GO:0031919], riboflavin transport [GO:0032218], alanine transport [GO:0032328], GO:0032329, 2-aminoethylphosphonate transport [GO:0033223], proline transmembrane transport [GO:0035524], amide transport [GO:0042886], GO:0042940, GO:0042968, daunorubicin transport [GO:0043215], azole transmembrane transport [GO:0045117], GO:0051470, histamine transport [GO:0051608], GO:0061528, octopamine secretion [GO:0061539], transepithelial ammonium transport [GO:0070634], modified amino acid transport [GO:0072337], ammonium transmembrane transport [GO:0072488], purine-containing compound transmembrane transport [GO:0072530], pyrimidine-containing compound transmembrane transport [GO:0072531], glutamate transmembrane import into vacuole [GO:0090454], sphingolipid translocation [GO:0099039], intermembrane sphingolipid transfer [GO:0120012], polyamine import across plasma membrane [GO:0140202], 5-aminolevulinic acid import across plasma membrane [GO:0140484], queuine import across plasma membrane [GO:0160284], GO:1900753, glucosinolate transport [GO:1901349], triazole transport [GO:1901504], GO:1902025, quinolinic acid transmembrane transport [GO:1903222], GO:1905329, GO:2001142 Sources: GOC:mah